protein localization to cilium [GO:0061512] (biological process) Regulation: regulated by regulation of protein localization to cilium [GO:1903564]; negatively regulated by negative regulation of protein localization to cilium [GO:1903565]; positively regulated by GO:1903566 Sources: GOC:dph Definition: A process in which a protein is transported to, or maintained in, a location within a cilium. Relationships: is a type of protein localization to organelle [GO:0033365] Subtypes: protein localization to non-motile cilium [GO:0097499], protein localization to motile cilium [GO:0120229], protein localization to ciliary membrane [GO:1903441], protein localization to ciliary inversin compartment [GO:1904108], protein localization to ciliary transition zone [GO:1904491]